{
  "term_label": "DNA damage response",
  "gene": "UniProtKB:Q96FW1",
  "term_id": "GO:0006974",
  "gene_symbol": "OTUB1",
  "gene_name": "Ubiquitin thioesterase OTUB1"
}